{
  "gene_name": "Semaphorin-3D",
  "term_label": "semaphorin receptor binding",
  "gene": "UniProtKB:O95025",
  "gene_symbol": "SEMA3D",
  "term_id": "GO:0030215"
}